{
  "term_id": "UNKNOWN:0001",
  "term_label": "Unknown molecular function",
  "gene_name": "Dynein axonemal assembly factor 9",
  "gene_symbol": "DNAAF9",
  "gene": "UniProtKB:Q5TEA3"
}